{
  "term_id": "GO:0001916",
  "term_label": "positive regulation of T cell mediated cytotoxicity",
  "gene_symbol": "ULBP2",
  "gene_name": "UL16-binding protein 2",
  "gene": "UniProtKB:Q9BZM5"
}